{
  "gene": "UniProtKB:Q92520",
  "term_id": "GO:0005615",
  "term_label": "extracellular space",
  "gene_name": "Protein FAM3C",
  "gene_symbol": "FAM3C"
}